{
  "gene_symbol": "IGF2BP1",
  "gene_name": "Insulin-like growth factor 2 mRNA-binding protein 1",
  "gene": "UniProtKB:Q9NZI8",
  "term_label": "nucleus",
  "term_id": "GO:0005634"
}